positive regulation of exosomal secretion [GO:1903543] (biological process) Relationships: is a type of positive regulation of cellular component biogenesis [GO:0044089]; is a type of GO:0045921; is a type of regulation of exosomal secretion [GO:1903541]; positively regulates exosomal secretion [GO:1990182] Also known as: positive regulation of exosomal secretory pathway, positive regulation of extracellular vesicular exosome secretion, positive regulation of secretion of exosome, up regulation of exosomal secretion, up regulation of exosomal secretory pathway, up regulation of extracellular vesicular exosome secretion, up regulation of secretion of exosome, up-regulation of exosomal secretion, up-regulation of exosomal secretory pathway, up-regulation of extracellular vesicular exosome secretion, up-regulation of secretion of exosome, upregulation of exosomal secretion, upregulation of exosomal secretory pathway, upregulation of extracellular vesicular exosome secretion, upregulation of secretion of exosome, activation of exosomal protein secretion, activation of exosomal secretion, activation of exosomal secretory pathway, activation of extracellular vesicular exosome secretion, activation of secretion of exosome, positive regulation of exosomal protein secretion, up regulation of exosomal protein secretion, up-regulation of exosomal protein secretion, upregulation of exosomal protein secretion Definition: Any process that activates or increases the frequency, rate or extent of exosomal secretion. References: PMID:24105262 Sources: GOC:TermGenie, GO_REF:0000058